{
  "gene_symbol": "TSLP",
  "term_label": "positive regulation of chemokine production",
  "gene": "UniProtKB:Q969D9",
  "gene_name": "Thymic stromal lymphopoietin",
  "term_id": "GO:0032722"
}